{
  "gene_symbol": "POU2AF2",
  "term_id": "GO:0043565",
  "term_label": "sequence-specific DNA binding",
  "gene_name": "POU domain class 2-associating factor 2",
  "gene": "UniProtKB:Q8IXP5"
}